{
  "gene_symbol": "TNFAIP3",
  "gene_name": "Tumor necrosis factor alpha-induced protein 3",
  "gene": "UniProtKB:P21580",
  "term_label": "ubiquitin-protein transferase activity",
  "term_id": "GO:0004842"
}